{
  "gene_symbol": "NANOGP1",
  "term_label": "nucleus",
  "term_id": "GO:0005634",
  "gene_name": "Putative homeobox protein NANOG2",
  "gene": "UniProtKB:Q8N7R0"
}